gamma-delta T cell differentiation involved in immune response [GO:0002303] (biological process) Note: Note that immunologists typically use the word 'development' to refer to cells of B or T cell lineages undergoing the process that GO describes as 'cell differentiation'. Definition: The process in which an antigenically naive gamma-delta T cell acquires the specialized features of an effector, regulatory, or memory T cell and contributes to an immune response. Effector T cells include cells which provide T cell help or exhibit cytotoxicity towards other cells. Sources: GOC:add Relationships: is a type of gamma-delta T cell activation involved in immune response [GO:0002290]; is a type of T cell differentiation involved in immune response [GO:0002292]; is a type of gamma-delta T cell differentiation [GO:0042492] Also known as: gamma-delta T cell development involved in immune response, gamma-delta T cell differentiation during immune response, gamma-delta T lymphocyte differentiation during immune response, gamma-delta T-cell differentiation during immune response, gamma-delta T-lymphocyte differentiation during immune response